{
  "term_id": "GO:0006368",
  "gene_symbol": "SUPT4H1",
  "gene_name": "Transcription elongation factor SPT4",
  "term_label": "transcription elongation by RNA polymerase II",
  "gene": "UniProtKB:P63272"
}